photoreceptor cell outer segment organization [GO:0035845] (BP) Definition: A process that is carried out at the cellular level and results in the assembly, arrangement of constituent parts, or disassembly of the outer segment of a photoreceptor cell, a sensory cell that reacts to the presence of light. The outer segment of the photoreceptor cell contains the light-absorbing materials. Also known as: photoreceptor cell outer segment organisation, photoreceptor outer segment organization References: PMID:14507858 Sources: ISBN:0824072820 Relationships: is a type of cellular component organization [GO:0016043]; is part of GO:0042461